{
  "term_id": "GO:0150007",
  "term_label": "clathrin-dependent synaptic vesicle endocytosis",
  "gene_symbol": "ITSN1",
  "gene_name": "Intersectin-1",
  "gene": "UniProtKB:Q15811"
}